{
  "term_id": "GO:0016339",
  "gene": "UniProtKB:Q9Y6N8",
  "gene_name": "Cadherin-10",
  "term_label": "calcium-dependent cell-cell adhesion",
  "gene_symbol": "CDH10"
}